terpenoid biosynthetic process, mevalonate-dependent [GO:0051485] (BP) Sources: GOC:ai Also known as: terpenoid anabolism, mevalonate-dependent, terpenoid formation, mevalonate-dependent, terpenoid synthesis, mevalonate-dependent, terpene biosynthesis, mevalonate-dependent, terpene biosynthetic process, mevalonate-dependent Definition: The chemical reactions and pathways resulting in the formation of terpenoids via isopentenyl diphosphate, synthesized by the mevalonate pathway. Isopentenyl diphosphate (IPP) is the fundamental unit in terpenoid biosynthesis, and in mevalonate-dependent terpenoid biosynthesis, acetate, in the form of acetyl-CoA, is converted to isopentenyl diphosphate (IPP) through a series of mevalonate intermediates. Relationships: is_a terpenoid biosynthetic process [GO:0016114]